{
  "gene_name": "Seizure 6-like protein 2",
  "term_id": "GO:0043025",
  "gene_symbol": "SEZ6L2",
  "term_label": "neuronal cell body",
  "gene": "UniProtKB:Q6UXD5"
}